heptadec-1-ene biosynthetic process [GO:1900875] (biological process) Also known as: heptadec-1-ene anabolism, heptadec-1-ene biosynthesis, heptadec-1-ene formation, heptadec-1-ene synthesis Sources: GOC:TermGenie, GOC:mengo_curators Definition: The chemical reactions and pathways resulting in the formation of heptadec-1-ene. Relationships: is a type of alkene biosynthetic process [GO:0043450]